{
  "term_id": "GO:0005886",
  "gene_name": "Olfactory receptor 2M5",
  "gene_symbol": "OR2M5",
  "term_label": "plasma membrane",
  "gene": "UniProtKB:A3KFT3"
}